{
  "gene_name": "Olfactory receptor 8B2",
  "gene": "UniProtKB:Q96RD0",
  "term_id": "GO:0007186",
  "term_label": "G protein-coupled receptor signaling pathway",
  "gene_symbol": "OR8B2"
}